oxidoreductase activity, acting on phosphorus or arsenic in donors, with NAD(P)+ as acceptor [GO:0050499] (MF) Sources: GOC:mah Relationships: is_a oxidoreductase activity, acting on phosphorus or arsenic in donors [GO:0030613] Subtypes: GO:0050609 Definition: Catalysis of an oxidation-reduction (redox) reaction in which a phosphorus- or arsenic-containing group acts as a hydrogen or electron donor and reduces a NAD(P)+ to NAD(P)H.